{
  "term_id": "GO:0006281",
  "gene": "UniProtKB:Q16531",
  "gene_symbol": "DDB1",
  "gene_name": "DNA damage-binding protein 1",
  "term_label": "DNA repair"
}